tRNA guanine ribose methylation [GO:0002938] (biological process) Relationships: is a type of GO:0002128 Sources: ISBN:1555811337 Subtypes: wobble position guanine ribose methylation [GO:0002129] Definition: The process whereby a guanosine residue in a tRNA is methylated on the 2'-hydroxyl group of the ribose moiety.